{
  "term_id": "GO:0005615",
  "gene_name": "Histone H2B type 1-O",
  "gene_symbol": "H2BC17",
  "gene": "UniProtKB:P23527",
  "term_label": "extracellular space"
}